{
  "gene_name": "BCLAF1 and THRAP3 family member 3",
  "term_label": "mediator complex",
  "gene": "UniProtKB:A2AJT9",
  "gene_symbol": "BCLAF3",
  "term_id": "GO:0016592"
}